determination of liver left/right asymmetry [GO:0071910] (biological process) Sources: GOC:cvs Definition: Determination of the asymmetric location of the liver with respect to the left and right halves of the organism. Relationships: is a type of GO:0007368; is part of liver development [GO:0001889]